{
  "gene_name": "Mitogen-activated protein kinase 8",
  "term_id": "GO:0004705",
  "gene": "UniProtKB:P45983",
  "gene_symbol": "MAPK8",
  "term_label": "JUN kinase activity"
}